{
  "term_label": "negative regulation of TOR signaling",
  "gene_name": "Glycogen synthase kinase-3 beta",
  "gene_symbol": "GSK3B",
  "term_id": "GO:0032007",
  "gene": "UniProtKB:P49841"
}